{
  "gene_symbol": "STX11",
  "gene_name": "Syntaxin-11",
  "gene": "UniProtKB:O75558",
  "term_label": "vesicle docking",
  "term_id": "GO:0048278"
}